{
  "gene": "UniProtKB:P42574",
  "gene_name": "Caspase-3",
  "term_label": "apoptotic process",
  "term_id": "GO:0006915",
  "gene_symbol": "CASP3"
}